{
  "gene": "UniProtKB:Q92908",
  "gene_symbol": "GATA6",
  "gene_name": "Transcription factor GATA-6",
  "term_label": "epithelial cell differentiation",
  "term_id": "GO:0030855"
}